{
  "gene": "UniProtKB:Q8IY63",
  "gene_name": "Angiomotin-like protein 1",
  "term_id": "UNKNOWN:0001",
  "term_label": "Unknown molecular function",
  "gene_symbol": "AMOTL1"
}